phospholipid transfer to membrane [GO:0006649] (biological process) Relationships: is a type of GO:0015914; is part of membrane organization [GO:0061024] Definition: The transfer of a phospholipid from its site of synthesis to the plasma membrane. Sources: GOC:go_curators